octanol metabolic process [GO:0006070] (biological process) Subtypes: octanol biosynthetic process [GO:0046171], octanol catabolic process [GO:0046172] Also known as: octanol metabolism Definition: The chemical reactions and pathways involving octanol, the 8-carbon alcohol with the formula C8H17OH. Sources: GOC:go_curators Relationships: is a type of primary alcohol metabolic process [GO:0034308]; is a type of fatty alcohol metabolic process [GO:1903173]